{
  "term_label": "axonemal basal plate",
  "term_id": "GO:0097541",
  "gene": "UniProtKB:O95876",
  "gene_name": "WD repeat-containing and planar cell polarity effector protein fritz homolog",
  "gene_symbol": "WDPCP"
}